{
  "term_label": "nucleus",
  "gene_symbol": "HIF3A",
  "gene_name": "Hypoxia-inducible factor 3-alpha",
  "gene": "UniProtKB:Q9Y2N7",
  "term_id": "GO:0005634"
}